{
  "gene_name": "Corticotropin-releasing factor receptor 1",
  "term_label": "neuron projection",
  "term_id": "GO:0043005",
  "gene": "UniProtKB:P34998",
  "gene_symbol": "CRHR1"
}